{
  "gene_name": "Integral membrane protein GPR180",
  "gene": "UniProtKB:Q86V85",
  "term_id": "UNKNOWN:0003",
  "term_label": "Unknown cellular component",
  "gene_symbol": "GPR180"
}